{
  "term_id": "UNKNOWN:0003",
  "gene": "UniProtKB:Q6TCH4",
  "gene_symbol": "PAQR6",
  "gene_name": "Membrane progestin receptor delta",
  "term_label": "Unknown cellular component"
}